{
  "gene_name": "General transcription and DNA repair factor IIH helicase subunit XPD",
  "gene_symbol": "ERCC2",
  "term_label": "positive regulation of mitotic recombination",
  "gene": "UniProtKB:P18074",
  "term_id": "GO:0045951"
}